interleukin-1 receptor antagonist activity [GO:0005152] (molecular function) Relationships: is a type of cytokine receptor binding [GO:0005126]; is a type of interleukin-1 binding [GO:0019966]; is a type of receptor antagonist activity [GO:0048019]; is part of negative regulation of cytokine-mediated signaling pathway [GO:0001960] Sources: GOC:ebc Also known as: IL-1ra Definition: Blocks the binding of interleukin-1 to the interleukin-1 receptor complex. Subtypes: interleukin-1 type I receptor antagonist activity [GO:0045352], interleukin-1 type II receptor antagonist activity [GO:0045353]